{
  "term_label": "regulation of transcription by RNA polymerase II",
  "gene_symbol": "BARHL2",
  "gene": "UniProtKB:Q9NY43",
  "term_id": "GO:0006357",
  "gene_name": "BarH-like 2 homeobox protein"
}